{
  "gene_name": "Fasciculation and elongation protein zeta-1",
  "term_label": "Unknown molecular function",
  "gene": "UniProtKB:Q99689",
  "gene_symbol": "FEZ1",
  "term_id": "UNKNOWN:0001"
}